regulation of oospore formation [GO:0075244] (biological process) Relationships: is_a regulation of sexual sporulation resulting in formation of a cellular spore [GO:0043940]; regulates GO:0075243 Sources: GOC:pamgo_curators Subtypes: positive regulation of oospore formation [GO:0075245], negative regulation of oospore formation [GO:0075246] Definition: Any process that modulates the frequency, rate or extent of oospore formation, a process in which male and female gametangia develop and fuse to form a thick-walled resting spore of oomycetes.